oligogalacturonide lyase activity [GO:0047487] (molecular function) Sources: EC:4.2.2.6, MetaCyc:OLIGOGALACTURONIDE-LYASE-RXN Definition: Catalysis of the reaction: 4-(4-deoxy-alpha-D-gluc-4-enuronosyl)-D-galacturonate = 2 5-dehydro-4-deoxy-D-glucuronate. Also known as: OGTE, oligogalacturonate lyase activity, unsaturated oligogalacturonate transeliminase activity Relationships: is a type of carbon-oxygen lyase activity, acting on polysaccharides [GO:0016837]